{
  "term_id": "GO:0000978",
  "gene_symbol": "BACH1",
  "gene": "UniProtKB:O14867",
  "gene_name": "Transcription regulator protein BACH1",
  "term_label": "RNA polymerase II cis-regulatory region sequence-specific DNA binding"
}